regulation of prostaglandin biosynthetic process [GO:0031392] (biological process) Relationships: is a type of GO:2001279; regulates prostaglandin biosynthetic process [GO:0001516] Definition: Any process that modulates the frequency, rate or extent of the chemical reactions and pathways resulting in the formation of prostaglandin. Sources: GOC:mah Also known as: regulation of prostaglandin anabolism, regulation of prostaglandin biosynthesis, regulation of prostaglandin formation, regulation of prostaglandin synthesis Subtypes: GO:0031393, positive regulation of prostaglandin biosynthetic process [GO:0031394], GO:0071809